membrane-oligosaccharide glycerophosphotransferase activity [GO:0047495] (molecular function) Also known as: periplasmic phosphoglycerotransferase activity, membrane-derived-oligosaccharide-6-(glycerophospho)-D-glucose:membrane-derived-oligosaccharide-D-glucose glycerophosphotransferase activity, phosphoglycerol cyclase activity Relationships: is a type of phosphotransferase activity, for other substituted phosphate groups [GO:0016780] Definition: Catalysis of the transfer of a glycerophospho group from one membrane-derived oligosaccharide to another. Sources: EC:2.7.8.21